{
  "term_id": "GO:0000775",
  "gene": "UniProtKB:P49454",
  "gene_symbol": "CENPF",
  "gene_name": "Centromere protein F",
  "term_label": "chromosome, centromeric region"
}